{
  "term_id": "UNKNOWN:0003",
  "gene_name": "Transmembrane protein 271",
  "gene_symbol": "TMEM271",
  "gene": "UniProtKB:A0A286YF58",
  "term_label": "Unknown cellular component"
}